{
  "term_id": "UNKNOWN:0003",
  "gene_name": "Uncharacterized protein C5orf52",
  "term_label": "Unknown cellular component",
  "gene_symbol": "C5orf52",
  "gene": "UniProtKB:A6NGY3"
}